{
  "gene_name": "Apolipoprotein C-III",
  "term_id": "GO:0034361",
  "gene_symbol": "APOC3",
  "term_label": "very-low-density lipoprotein particle",
  "gene": "UniProtKB:P02656"
}